medium-chain fatty acyl-CoA hydrolase activity [GO:0052815] (molecular function) Note: While there is not universal consensus on the lengths of short-, medium-, long- and very-long-chain fatty acids, the GO uses the definitions in ChEBI (see CHEBI:26666, CHEBI:59554, CHEBI:15904 and CHEBI:27283). Definition: Catalysis of the reaction: a medium-chain fatty acyl-CoA + H2O = a medium-chain fatty acid + CoA + H+. A medium-chain fatty acid has an aliphatic tail containing 6 to 12 carbons. Also known as: medium-chain acyl coenzyme A hydrolase activity, medium-chain acyl-thioester hydrolase activity, medium-chain hydrolase activity, medium-chain-acyl-CoA hydrolase activity Sources: RHEA:68184 Relationships: is a type of fatty acyl-CoA hydrolase activity [GO:0047617]